{
  "term_label": "DNA-binding transcription factor activity, RNA polymerase II-specific",
  "gene_symbol": "FOXD4L3",
  "gene_name": "Forkhead box protein D4-like 3",
  "term_id": "GO:0000981",
  "gene": "UniProtKB:Q6VB84"
}